{
  "gene_name": "Neurotrophin receptor-interacting factor homolog",
  "term_id": "GO:0000981",
  "gene_symbol": "ZNF274",
  "gene": "UniProtKB:Q96GC6",
  "term_label": "DNA-binding transcription factor activity, RNA polymerase II-specific"
}